{
  "gene_symbol": "URGCP",
  "term_id": "UNKNOWN:0002",
  "gene_name": "Up-regulator of cell proliferation",
  "term_label": "Unknown biological process",
  "gene": "UniProtKB:Q8TCY9"
}